{
  "gene_name": "Nuclear receptor subfamily 0 group B member 1",
  "term_label": "spermatogenesis",
  "gene": "UniProtKB:P51843",
  "term_id": "GO:0007283",
  "gene_symbol": "NR0B1"
}